{
  "term_id": "GO:0007265",
  "gene_name": "RAS guanyl-releasing protein 2",
  "gene_symbol": "RASGRP2",
  "gene": "UniProtKB:Q7LDG7",
  "term_label": "Ras protein signal transduction"
}